{
  "gene_symbol": "PTCHD4",
  "term_label": "membrane",
  "gene": "UniProtKB:Q6ZW05",
  "gene_name": "Patched domain-containing protein 4",
  "term_id": "GO:0016020"
}